{
  "gene_name": "Transmembrane 9 superfamily member 3",
  "term_id": "UNKNOWN:0001",
  "term_label": "Unknown molecular function",
  "gene_symbol": "TM9SF3",
  "gene": "UniProtKB:Q9HD45"
}